{
  "gene": "UniProtKB:Q9NVF7",
  "gene_symbol": "FBXO28",
  "term_label": "Unknown molecular function",
  "term_id": "UNKNOWN:0001",
  "gene_name": "F-box only protein 28"
}